cyclization of asparagine involved in intein-mediated protein splicing [GO:0019801] (biological process) Definition: The cyclization of asparagine to yield an L-aspartimide (otherwise known as alpha-aminosuccinimide) residue at the C-terminus of an excised intein during protein splicing. Relationships: is a type of asparagine metabolic process [GO:0006528]; is part of intein-mediated protein splicing [GO:0016539] Note: See also the biological process term 'intein-mediated protein splicing ; GO:0016539'. Also known as: cyclization of asparagine, during protein splicing Sources: RESID:AA0302